{
  "term_label": "nucleus",
  "term_id": "GO:0005634",
  "gene_symbol": "PNO1",
  "gene_name": "RNA-binding protein PNO1",
  "gene": "UniProtKB:Q9NRX1"
}